{
  "gene": "UniProtKB:Q9UHY8",
  "gene_symbol": "FEZ2",
  "term_label": "Unknown biological process",
  "gene_name": "Fasciculation and elongation protein zeta-2",
  "term_id": "UNKNOWN:0002"
}